{
  "gene": "UniProtKB:Q8WUY9",
  "term_label": "positive regulation of Wnt signaling pathway",
  "gene_symbol": "DEPDC1B",
  "term_id": "GO:0030177",
  "gene_name": "DEP domain-containing protein 1B"
}